collagen type VI trimer [GO:0005589] (CC) Relationships: is a type of von-Willerbrand-factor-A-domain-rich collagen trimer [GO:0140158]; is part of collagen beaded filament [GO:0098647] References: PMID:19693541, PMID:21421911 Definition: A collagen heterotrimer containing type VI alpha chains in alpha1(VI)alpha2(VI)alpha3(VI) trimers; type VI collagen triple helices associate to form beaded fibrils.